sulfide oxidation, using sulfide:quinone oxidoreductase [GO:0070221] (biological process) Definition: A sulfide oxidation process that proceeds via the reaction catalyzed by sulfide:quinone oxidoreductase. Relationships: is a type of sulfide oxidation [GO:0019418] Also known as: sulfide oxidation, using sulfide-quinone reductase, sulphide oxidation, using sulfide:quinone oxidoreductase Sources: MetaCyc:P222-PWY